{
  "term_id": "GO:0032391",
  "term_label": "photoreceptor connecting cilium",
  "gene": "UniProtKB:Q3SY00",
  "gene_symbol": "TSGA10IP",
  "gene_name": "Testis-specific protein 10-interacting protein"
}